{
  "gene_symbol": "JAK1",
  "gene": "UniProtKB:P23458",
  "term_label": "non-membrane spanning protein tyrosine kinase activity",
  "gene_name": "Tyrosine-protein kinase JAK1",
  "term_id": "GO:0004715"
}